{
  "gene_name": "Tripartite motif-containing protein 49",
  "gene": "UniProtKB:P0CI25",
  "gene_symbol": "TRIM49",
  "term_id": "GO:0061630",
  "term_label": "ubiquitin protein ligase activity"
}